{
  "gene_name": "Hairy_enhancer-of-split related with YRPW motif protein 1",
  "gene": "UniProtKB:Q9Y5J3",
  "gene_symbol": "HEY1",
  "term_id": "GO:0045665",
  "term_label": "negative regulation of neuron differentiation"
}